chlordecone reductase activity [GO:0047743] (molecular function) Definition: Catalysis of the reaction: chlordecone alcohol + NADP+ = chlordecone + H+ + NADPH. Sources: EC:1.1.1.225, RHEA:14401 Also known as: CDR activity, chlordecone-alcohol:NADP+ 2-oxidoreductase activity Relationships: is a type of oxidoreductase activity, acting on the CH-OH group of donors, NAD or NADP as acceptor [GO:0016616]